regulation of oligodendrocyte apoptotic process [GO:1900141] (biological process) Definition: Any process that modulates the frequency, rate or extent of oligodendrocyte apoptotic process. Subtypes: negative regulation of oligodendrocyte apoptotic process [GO:1900142], GO:1900143 Sources: GOC:TermGenie, GOC:yaf Relationships: is a type of regulation of glial cell apoptotic process [GO:0034350]; regulates GO:0097252 Also known as: regulation of oligodendrocyte apoptosis